dimethylsulfoniopropionate catabolic process [GO:1902087] (biological process) Definition: The chemical reactions and pathways resulting in the breakdown of S,S-dimethyl-beta-propiothetin. References: PMID:19807777 Sources: GOC:TermGenie, GOC:jh2 Also known as: S,S-dimethyl-beta-propiothetin breakdown, S,S-dimethyl-beta-propiothetin catabolic process, S,S-dimethyl-beta-propiothetin catabolism, S,S-dimethyl-beta-propiothetin degradation Relationships: is a type of sulfur compound catabolic process [GO:0044273]